rejection of self pollen [GO:0060320] (BP) References: PMID:34848142 Sources: GOC:dph, GOC:tb Relationships: is a type of recognition of pollen [GO:0048544] Also known as: self-incompatibility Definition: The recognition and rejection of self pollen by cells in the stigma, mediated by the sharing and interaction of the single locus incompatibility haplotypes.